{
  "gene": "UniProtKB:P59095",
  "gene_symbol": "STARD6",
  "gene_name": "StAR-related lipid transfer protein 6",
  "term_label": "Unknown cellular component",
  "term_id": "UNKNOWN:0003"
}